{
  "term_id": "GO:0009617",
  "gene": "UniProtKB:A0A0B4J275",
  "gene_symbol": "TRAV17",
  "gene_name": "T cell receptor alpha variable 17",
  "term_label": "response to bacterium"
}